{
  "gene": "UniProtKB:P55058",
  "term_id": "GO:0120017",
  "gene_symbol": "PLTP",
  "term_label": "ceramide transfer activity",
  "gene_name": "Phospholipid transfer protein"
}